{
  "term_id": "GO:0000981",
  "term_label": "DNA-binding transcription factor activity, RNA polymerase II-specific",
  "gene_name": "Cyclic AMP-dependent transcription factor ATF-6 beta",
  "gene": "UniProtKB:Q99941",
  "gene_symbol": "ATF6B"
}